{
  "gene": "UniProtKB:O14530",
  "gene_symbol": "TXNDC9",
  "term_id": "GO:0005737",
  "term_label": "cytoplasm",
  "gene_name": "Thioredoxin domain-containing protein 9"
}